{
  "gene_name": "Homeobox protein prophet of Pit-1",
  "gene": "UniProtKB:O75360",
  "gene_symbol": "PROP1",
  "term_label": "RNA polymerase II cis-regulatory region sequence-specific DNA binding",
  "term_id": "GO:0000978"
}